{
  "term_id": "GO:0051864",
  "gene_symbol": "KDM4A",
  "gene_name": "Lysine-specific demethylase 4A",
  "gene": "UniProtKB:O75164",
  "term_label": "histone H3K36 demethylase activity"
}